{
  "gene_name": "ADP-ribosylation factor-like protein 4C",
  "gene": "UniProtKB:P56559",
  "term_id": "GO:0005525",
  "gene_symbol": "ARL4C",
  "term_label": "GTP binding"
}